{
  "gene_name": "Zona pellucida sperm-binding protein 4",
  "term_id": "GO:0060468",
  "gene_symbol": "ZP4",
  "gene": "UniProtKB:Q12836",
  "term_label": "prevention of polyspermy"
}